{
  "term_label": "polar microtubule",
  "gene": "UniProtKB:Q53GT1",
  "term_id": "GO:0005827",
  "gene_symbol": "KLHL22",
  "gene_name": "Kelch-like protein 22"
}